{
  "gene_symbol": "LETM2",
  "gene": "UniProtKB:Q2VYF4",
  "gene_name": "LETM1 domain-containing protein LETM2, mitochondrial",
  "term_label": "transmembrane transporter activity",
  "term_id": "GO:0022857"
}